negative regulation of lung blood pressure [GO:0061767] (biological process) Relationships: is a type of regulation of lung blood pressure [GO:0014916] Also known as: negative regulation of pulmonary blood pressure References: PMID:22161164 Sources: GOC:BHF, GOC:BHF_miRNA, GOC:bc, GOC:dph Definition: The process that decreases the force with which blood travels through the lungs.